{
  "gene": "UniProtKB:P17787",
  "gene_symbol": "CHRNB2",
  "gene_name": "Neuronal acetylcholine receptor subunit beta-2",
  "term_label": "neuron projection",
  "term_id": "GO:0043005"
}